{
  "term_id": "GO:0019221",
  "gene_name": "Interleukin-1 alpha",
  "gene_symbol": "IL1A",
  "term_label": "cytokine-mediated signaling pathway",
  "gene": "UniProtKB:P01583"
}